{
  "term_label": "extracellular space",
  "gene": "UniProtKB:O43508",
  "gene_symbol": "TNFSF12",
  "term_id": "GO:0005615",
  "gene_name": "Tumor necrosis factor ligand superfamily member 12"
}